{
  "gene": "UniProtKB:Q9H4Y5",
  "gene_name": "Glutathione S-transferase omega-2",
  "gene_symbol": "GSTO2",
  "term_id": "GO:0005737",
  "term_label": "cytoplasm"
}